{
  "term_id": "UNKNOWN:0001",
  "term_label": "Unknown molecular function",
  "gene_symbol": "FAM168B",
  "gene_name": "Myelin-associated neurite-outgrowth inhibitor",
  "gene": "UniProtKB:A1KXE4"
}